{
  "term_id": "UNKNOWN:0001",
  "gene": "UniProtKB:H0UI37",
  "gene_name": "Thiosulfate sulfurtransferase_rhodanese-like domain-containing protein 3",
  "term_label": "Unknown molecular function",
  "gene_symbol": "TSTD3"
}